spinal cord ventral commissure morphogenesis [GO:0021965] (biological process) Definition: The process in which the anatomical structures of the spinal cord ventral commissure are generated and organized. Relationships: is_a GO:0021952; is part of spinal cord development [GO:0021510] Sources: GOC:cls, GOC:dgh, GOC:dph, GOC:jid, GO_REF:0000021